{
  "gene": "UniProtKB:P57103",
  "term_id": "GO:0035725",
  "gene_name": "Sodium_calcium exchanger 3",
  "gene_symbol": "SLC8A3",
  "term_label": "sodium ion transmembrane transport"
}